{
  "term_id": "UNKNOWN:0001",
  "gene": "UniProtKB:A6NMK7",
  "gene_symbol": "CPSF4L",
  "gene_name": "Putative cleavage and polyadenylation specificity factor subunit 4-like protein",
  "term_label": "Unknown molecular function"
}